{
  "gene_symbol": "KLK5",
  "gene_name": "Kallikrein-5",
  "gene": "UniProtKB:Q9Y337",
  "term_id": "GO:0097186",
  "term_label": "amelogenesis"
}